{
  "term_label": "positive regulation of neuron apoptotic process",
  "gene_symbol": "CASP4",
  "gene_name": "Caspase-4",
  "term_id": "GO:0043525",
  "gene": "UniProtKB:P49662"
}